{
  "gene_symbol": "DCLK3",
  "gene_name": "Serine_threonine-protein kinase DCLK3",
  "term_id": "GO:0004674",
  "gene": "UniProtKB:Q9C098",
  "term_label": "protein serine/threonine kinase activity"
}